regulation of butyryl-CoA catabolic process to butanol [GO:1900497] (biological process) Also known as: regulation of butyryl-CoA catabolism to butanol Sources: GOC:TermGenie, GOC:mengo_curators Subtypes: negative regulation of butyryl-CoA catabolic process to butanol [GO:1900498], GO:1900499 Relationships: is a type of regulation of fatty acid metabolic process [GO:0019217]; is a type of regulation of nucleobase-containing compound metabolic process [GO:0019219]; is a type of regulation of amide metabolic process [GO:0034248]; is a type of regulation of sulfur metabolic process [GO:0042762]; is a type of regulation of lipid biosynthetic process [GO:0046890]; is a type of regulation of lipid catabolic process [GO:0050994]; is a type of regulation of phosphorus metabolic process [GO:0051174]; is a type of GO:1902930; regulates butyryl-CoA catabolic process to butanol [GO:0044582] Definition: Any process that modulates the frequency, rate or extent of butyryl-CoA catabolic process to butanol.